iNOS-S100A8/A9 complex [GO:1990657] (cellular component) References: PMID:25417112 Sources: GOC:bhm Definition: A protein complex capable of stimulus-inducible nitric-oxide synthase activity. S-nitrosylates cysteine residues in target proteins, a principal mechanism of nitric oxide (NO)-mediated signal transduction. In mammals consists of NOS2, S100A8 and S100A9. S100A9 acts both as an adaptor linking NOS2 to its target and as a transnitrosylase that transfers the nitric oxide moiety from NOS2 to its target, via its own S-nitrosylated cysteine. Note: An example of this is NOS2 in human (UniProt symbol P35228) in PMID:25417112 (inferred from direct assay). Relationships: is a type of nitric-oxide synthase complex [GO:1903958]; is a type of transnitrosylase complex [GO:1990658]